{
  "gene": "UniProtKB:Q92504",
  "gene_symbol": "SLC39A7",
  "term_label": "intracellular zinc ion homeostasis",
  "gene_name": "Zinc transporter SLC39A7",
  "term_id": "GO:0006882"
}